regulation of translational initiation in response to starvation [GO:0071262] (biological process) Sources: GOC:mah Also known as: regulation of translational initiation in response to nutrient starvation Subtypes: GO:0071263, positive regulation of translational initiation in response to starvation [GO:0071264] Definition: Any process that modulates the frequency, rate or extent of translation initiation, as a result of deprivation of nourishment. Relationships: is a type of regulation of translational initiation in response to stress [GO:0043558]; is part of cellular response to starvation [GO:0009267]